somal translocation [GO:0021802] (biological process) Definition: The radial migration of cells from the ventricular zone that is independent of radial glial cells. Cells extend processes that terminate at the pial surface and follow the processes as they migrate. References: PMID:12626695 Sources: GOC:cls, GOC:dgh, GOC:dph, GOC:jid, GO_REF:0000021 Also known as: perikaryal translocation of Morest Relationships: is a type of GO:0021799